{
  "gene": "UniProtKB:P00742",
  "gene_name": "Coagulation factor X",
  "term_label": "serine-type endopeptidase activity",
  "gene_symbol": "F10",
  "term_id": "GO:0004252"
}